{
  "term_label": "neurotransmitter receptor activity",
  "gene_name": "D(4) dopamine receptor",
  "term_id": "GO:0030594",
  "gene": "UniProtKB:P21917",
  "gene_symbol": "DRD4"
}